regulation of secondary heart field cardioblast proliferation [GO:0003266] (biological process) Subtypes: positive regulation of secondary heart field cardioblast proliferation [GO:0072513] Definition: Any process that modulates the frequency, rate or extent of cardioblast proliferation in the second heart field. A cardioblast is a cardiac precursor cell. It is a cell that has been committed to a cardiac fate, but will undergo more cell division rather than terminally differentiating. The secondary heart field is the region of the heart that will form the majority of the mesodermal component of the right ventricle, the arterial pole (outflow tract) and the venous pole (inflow tract). Also known as: regulation of SHF cardioblast proliferation, regulation of second heart field cardioblast proliferation Relationships: is_a regulation of cardioblast proliferation [GO:0003264] References: PMID:17276708 Sources: GOC:mtg_heart, GOC:rl